solute:potassium antiporter activity [GO:0022821] (molecular function) Relationships: is_a potassium ion transmembrane transporter activity [GO:0015079]; is a type of metal cation:monoatomic cation antiporter activity [GO:0140828] Sources: GOC:mtg_transport, ISBN:0815340729 Also known as: potassium ion antiporter activity Subtypes: calcium, potassium:sodium antiporter activity [GO:0008273], GO:0015386, GO:0015503 Definition: Catalysis of the active transport of a potassium ion across a membrane by a mechanism whereby two or more species are transported in opposite directions in a tightly coupled process not directly linked to a form of energy other than chemiosmotic energy.